{
  "gene_symbol": "SLC39A14",
  "term_id": "GO:0140410",
  "gene_name": "Metal cation symporter ZIP14",
  "gene": "UniProtKB:Q15043",
  "term_label": "monoatomic cation:bicarbonate symporter activity"
}